{
  "gene_name": "Protein arginine N-methyltransferase 8",
  "gene": "UniProtKB:Q9NR22",
  "term_label": "chromatin remodeling",
  "gene_symbol": "PRMT8",
  "term_id": "GO:0006338"
}